host cell nuclear part [GO:0044094] (cellular component) Subtypes: GO:0019034, host cell nucleoplasm [GO:0044095], host cell nucleolus [GO:0044196], host cell nuclear envelope [GO:0044199], host cell nuclear lamina [GO:0044203], host cell nuclear matrix [GO:0044204], host cell Cajal body [GO:0072495], GO:0075341 Definition: Any constituent part of a host cell's nucleus, a membrane-bounded organelle of eukaryotic cells in which chromosomes are housed and replicated. The host is the larger of the organisms involved in a symbiotic interaction. Note: Note that this term is in the subset of terms that should not be used for direct gene product annotation. Instead, select a child term or, if no appropriate child term exists, please request a new term. Direct annotations to this term may be amended during annotation QC. Relationships: is a type of host intracellular part [GO:0033646]; is part of host cell nucleus [GO:0042025] Sources: GOC:ecd